{
  "term_label": "GTPase activity",
  "gene_name": "Arf-GAP with GTPase, ANK repeat and PH domain-containing protein 3",
  "term_id": "GO:0003924",
  "gene_symbol": "AGAP3",
  "gene": "UniProtKB:Q96P47"
}